carbohydrate metabolic process [GO:0005975] (biological process) Regulation: regulated by GO:0006109; negatively regulated by GO:0045912; RO_0002213 by GO:0045913 Definition: The chemical reactions and pathways involving carbohydrates, any of a group of organic compounds based of the general formula Cx(H2O)y. Subtypes: polysaccharide metabolic process [GO:0005976], monosaccharide metabolic process [GO:0005996], hexitol metabolic process [GO:0006059], GO:0006071, GO:0006097, oligosaccharide metabolic process [GO:0009311], carbohydrate biosynthetic process [GO:0016051], GO:0016052, GO:0019519, D-gluconate metabolic process [GO:0019521], D-glucarate metabolic process [GO:0042836], carbohydrate phosphorylation [GO:0046835], mannosylglycerate metabolic process [GO:0051478] Also known as: carbohydrate metabolism Relationships: is a type of GO:0044238 Sources: GOC:mah, ISBN:0198506732